osmolarity-sensing monoatomic cation channel activity [GO:1990760] (molecular function) Also known as: osmolarity-sensing cation channel activity References: PMID:18279313 Definition: Enables the transmembrane transfer of a monoatomic cation by a channel that opens when a change in the osmolarity occurs in the extracellular space of the cell in which the cation channel resides. Relationships: is a type of osmosensor activity [GO:0005034]; is a type of GO:0005261; is a type of gated channel activity [GO:0022836]